steroid dehydrogenase activity, acting on the CH-CH group of donors [GO:0033765] (molecular function) Relationships: is a type of steroid dehydrogenase activity [GO:0016229]; is a type of oxidoreductase activity, acting on the CH-CH group of donors [GO:0016627] Sources: GOC:mah Subtypes: 3-oxo-5-alpha-steroid 4-dehydrogenase activity [GO:0003865], GO:0047568, 3-oxosteroid 1-dehydrogenase activity [GO:0047571] Definition: Catalysis of an oxidation-reduction (redox) reaction in which a CH-CH group acts as a hydrogen or electron donor and reduces a hydrogen or electron acceptor, and in which one substrate is a sterol derivative.